{
  "gene": "UniProtKB:Q9Y5G7",
  "term_id": "GO:0050839",
  "gene_symbol": "PCDHGA6",
  "gene_name": "Protocadherin gamma-A6",
  "term_label": "cell adhesion molecule binding"
}